{
  "gene_name": "Sarcospan",
  "gene": "UniProtKB:Q14714",
  "term_label": "Unknown biological process",
  "term_id": "UNKNOWN:0002",
  "gene_symbol": "SSPN"
}